{
  "term_id": "UNKNOWN:0001",
  "gene": "UniProtKB:P31944",
  "gene_symbol": "CASP14",
  "term_label": "Unknown molecular function",
  "gene_name": "Caspase-14"
}